{
  "term_label": "endoplasmic reticulum-Golgi intermediate compartment",
  "term_id": "GO:0005793",
  "gene_name": "Transmembrane emp24 domain-containing protein 4",
  "gene_symbol": "TMED4",
  "gene": "UniProtKB:Q7Z7H5"
}